{
  "gene_symbol": "PITPNB",
  "term_label": "cytoplasm",
  "gene_name": "Phosphatidylinositol transfer protein beta isoform",
  "term_id": "GO:0005737",
  "gene": "UniProtKB:P48739"
}